nuclear-transcribed mRNA catabolic process, no-go decay [GO:0070966] (biological process) Definition: The chemical reactions and pathways resulting in the breakdown of the transcript body of a nuclear-transcribed mRNA with stalls in translation elongation. References: PMID:16554824 Sources: GOC:jp Also known as: no-go decay, no-go mRNA decay, nuclear-transcribed mRNA breakdown, no-go decay, nuclear-transcribed mRNA catabolism, no-go decay, nuclear-transcribed mRNA degradation, no-go decay Relationships: is a type of nuclear-transcribed mRNA catabolic process [GO:0000956]